{
  "term_id": "GO:0033041",
  "gene_symbol": "TAS1R3",
  "term_label": "sweet taste receptor activity",
  "gene": "UniProtKB:Q7RTX0",
  "gene_name": "Taste receptor type 1 member 3"
}